MCM core complex [GO:0097373] (CC) Definition: A protein complex that contains Mcm4, Mcm6, and Mcm7 proteins, and possesses DNA helicase activity. In the heterohexameric MCM complex, the Mcm4/6/7 proteins form a stable core, and Mcm2, Mcm3, and Mcm5 are more peripherally associated. References: PMID:10770926, PMID:15007098, PMID:9305914 Sources: GOC:mah Also known as: MCM4/6/7 complex Relationships: is a type of protein-containing complex [GO:0032991]